{
  "gene_name": "Protein BTG4",
  "gene": "UniProtKB:Q9NY30",
  "term_label": "nucleus",
  "gene_symbol": "BTG4",
  "term_id": "GO:0005634"
}